{
  "term_id": "UNKNOWN:0002",
  "term_label": "Unknown biological process",
  "gene": "UniProtKB:Q8IZ83",
  "gene_name": "Aldehyde dehydrogenase family 16 member A1",
  "gene_symbol": "ALDH16A1"
}